{
  "gene_symbol": "ADORA2A-AS1",
  "gene": "UniProtKB:P86434",
  "term_label": "Unknown biological process",
  "term_id": "UNKNOWN:0002",
  "gene_name": "Putative uncharacterized protein ADORA2A-AS1"
}